{
  "gene_name": "Phosphorylase b kinase gamma catalytic chain, liver_testis isoform",
  "term_label": "glycogen metabolic process",
  "term_id": "GO:0005977",
  "gene_symbol": "PHKG2",
  "gene": "UniProtKB:P15735"
}